{
  "gene": "UniProtKB:P23229",
  "gene_name": "Integrin alpha-6",
  "term_label": "signaling receptor activity",
  "gene_symbol": "ITGA6",
  "term_id": "GO:0038023"
}